{
  "gene_symbol": "SHISA3",
  "gene": "UniProtKB:A0PJX4",
  "term_id": "UNKNOWN:0001",
  "term_label": "Unknown molecular function",
  "gene_name": "Protein shisa-3 homolog"
}